{
  "term_label": "serine-type endopeptidase activity",
  "gene": "UniProtKB:P17538",
  "gene_symbol": "CTRB1",
  "term_id": "GO:0004252",
  "gene_name": "Chymotrypsinogen B"
}